{
  "gene_name": "Annexin A13",
  "term_id": "GO:0005886",
  "gene": "UniProtKB:P27216",
  "gene_symbol": "ANXA13",
  "term_label": "plasma membrane"
}